{
  "term_id": "GO:0001817",
  "gene": "UniProtKB:Q96KV6",
  "gene_name": "Putative butyrophilin subfamily 2 member A3",
  "term_label": "regulation of cytokine production",
  "gene_symbol": "BTN2A3P"
}